{
  "term_id": "UNKNOWN:0002",
  "gene_symbol": "SNTG1",
  "gene": "UniProtKB:Q9NSN8",
  "term_label": "Unknown biological process",
  "gene_name": "Gamma-1-syntrophin"
}